response to fungicide [GO:0060992] (biological process) Definition: Any process that results in a change in state or activity of a cell or an organism (in terms of movement, secretion, enzyme production, gene expression, etc.) as a result of a fungicide stimulus. Fungicides are chemicals used to kill fungi. Sources: GOC:dph Relationships: is a type of response to toxic substance [GO:0009636]; is a type of response to antibiotic [GO:0046677]